{
  "gene_symbol": "NTNG2",
  "term_id": "GO:0005886",
  "gene": "UniProtKB:Q96CW9",
  "gene_name": "Netrin-G2",
  "term_label": "plasma membrane"
}